{
  "gene_name": "Folliculin-interacting protein 1",
  "term_label": "cytoplasm",
  "term_id": "GO:0005737",
  "gene": "UniProtKB:Q8TF40",
  "gene_symbol": "FNIP1"
}